{
  "gene_symbol": "PLA2G10",
  "gene": "UniProtKB:O15496",
  "term_id": "UNKNOWN:0003",
  "gene_name": "Group 10 secretory phospholipase A2",
  "term_label": "Unknown cellular component"
}